{
  "term_id": "GO:1990756",
  "gene_name": "Protein fem-1 homolog B",
  "gene_symbol": "FEM1B",
  "gene": "UniProtKB:Q9UK73",
  "term_label": "ubiquitin-like ligase-substrate adaptor activity"
}